{
  "gene_name": "Uncharacterized protein C11orf91",
  "term_label": "Unknown biological process",
  "gene_symbol": "C11orf91",
  "gene": "UniProtKB:Q3C1V1",
  "term_id": "UNKNOWN:0002"
}